alpha-D-glucan binding [GO:2001083] (molecular function) Definition: Binding to alpha-D-glucan. Sources: GOC:mengo_curators Relationships: is a type of polysaccharide binding [GO:0030247]